{
  "term_label": "U1 snRNP",
  "gene_symbol": "SNRNP70",
  "gene": "UniProtKB:P08621",
  "term_id": "GO:0005685",
  "gene_name": "U1 small nuclear ribonucleoprotein 70 kDa"
}